anterior/posterior pattern specification involved in kidney development [GO:0072098] (BP) Definition: The developmental process that results in the creation of defined areas or spaces within the kidney along the anterior/posterior axis to which cells respond and eventually are instructed to differentiate. Also known as: kidney anterior/posterior pattern specification, anterior/posterior pattern formation involved in kidney development, kidney anterior/posterior pattern formation Relationships: is a type of anterior/posterior pattern specification [GO:0009952]; is a type of pattern specification involved in kidney development [GO:0061004] Sources: GOC:mtg_kidney_jan10 Subtypes: GO:0034672, anterior/posterior pattern specification involved in ureteric bud development [GO:0072099], GO:0072168, specification of posterior mesonephric tubule identity [GO:0072169]